{
  "gene_symbol": "TBR1",
  "gene_name": "T-box brain protein 1",
  "term_label": "regulation of neuron projection development",
  "gene": "UniProtKB:Q16650",
  "term_id": "GO:0010975"
}